{
  "gene": "UniProtKB:Q9ULY5",
  "term_label": "external side of plasma membrane",
  "gene_symbol": "CLEC4E",
  "gene_name": "C-type lectin domain family 4 member E",
  "term_id": "GO:0009897"
}